{
  "gene_name": "Prolow-density lipoprotein receptor-related protein 1",
  "gene": "UniProtKB:Q07954",
  "gene_symbol": "LRP1",
  "term_label": "amyloid-beta clearance by cellular catabolic process",
  "term_id": "GO:0150094"
}